serine O-acetyltransferase activity [GO:0009001] (molecular function) Sources: RHEA:24560 Definition: Catalysis of the reaction: L-serine + acetyl-CoA = O-acetyl-L-serine + CoA. Also known as: L-serine acetyltransferase activity, SATase activity, acetyl-CoA:L-serine O-acetyltransferase activity, serine acetyltransferase activity, serine transacetylase activity Relationships: is a type of serine O-acyltransferase activity [GO:0016412]; is a type of O-acetyltransferase activity [GO:0016413]